{
  "gene": "UniProtKB:Q86V86",
  "gene_name": "Serine_threonine-protein kinase pim-3",
  "term_id": "GO:0043066",
  "gene_symbol": "PIM3",
  "term_label": "negative regulation of apoptotic process"
}